{
  "term_id": "GO:0010764",
  "gene_symbol": "MACIR",
  "gene": "UniProtKB:Q96GV9",
  "term_label": "negative regulation of fibroblast migration",
  "gene_name": "Macrophage immunometabolism regulator"
}